{
  "term_id": "GO:0004713",
  "gene": "UniProtKB:Q8NE63",
  "term_label": "protein tyrosine kinase activity",
  "gene_symbol": "HIPK4",
  "gene_name": "Homeodomain-interacting protein kinase 4"
}